{
  "term_label": "inflammatory response",
  "term_id": "GO:0006954",
  "gene": "UniProtKB:O15444",
  "gene_symbol": "CCL25",
  "gene_name": "C-C motif chemokine 25"
}